{
  "gene_symbol": "SUSD5",
  "term_label": "Unknown molecular function",
  "gene": "UniProtKB:O60279",
  "gene_name": "Sushi domain-containing protein 5",
  "term_id": "UNKNOWN:0001"
}